{
  "term_id": "GO:0031005",
  "gene": "UniProtKB:Q8WUP2",
  "gene_name": "Filamin-binding LIM protein 1",
  "gene_symbol": "FBLIM1",
  "term_label": "filamin binding"
}